{
  "gene": "UniProtKB:Q9Y547",
  "gene_name": "Intraflagellar transport protein 25 homolog",
  "term_id": "GO:0030992",
  "term_label": "intraciliary transport particle B",
  "gene_symbol": "IFT25"
}